{
  "gene": "UniProtKB:Q9UBD9",
  "term_id": "GO:0097059",
  "term_label": "CNTFR-CLCF1 complex",
  "gene_name": "Cardiotrophin-like cytokine factor 1",
  "gene_symbol": "CLCF1"
}